{
  "gene": "UniProtKB:Q16254",
  "term_label": "RNA polymerase II cis-regulatory region sequence-specific DNA binding",
  "term_id": "GO:0000978",
  "gene_symbol": "E2F4",
  "gene_name": "Transcription factor E2F4"
}